{
  "gene": "UniProtKB:P35749",
  "term_label": "microfilament motor activity",
  "gene_symbol": "MYH11",
  "gene_name": "Myosin-11",
  "term_id": "GO:0000146"
}